wax metabolic process [GO:0010166] (biological process) Sources: GOC:sm Definition: The chemical reactions and pathways involving wax, a compound containing C16 and C18 fatty acids. Subtypes: GO:0010025 Also known as: wax metabolism Relationships: is a type of fatty acid derivative metabolic process [GO:1901568]